{
  "term_label": "B cell activation involved in immune response",
  "gene_name": "Interferon alpha-21",
  "gene": "UniProtKB:P01568",
  "gene_symbol": "IFNA21",
  "term_id": "GO:0002312"
}